{
  "term_id": "GO:0003677",
  "gene_symbol": "SMARCA1",
  "term_label": "DNA binding",
  "gene": "UniProtKB:P28370",
  "gene_name": "Probable global transcription activator SNF2L1"
}